{
  "term_label": "3'-5'-DNA exonuclease activity",
  "gene_name": "Three prime repair exonuclease 2",
  "term_id": "GO:0008296",
  "gene": "UniProtKB:Q9BQ50",
  "gene_symbol": "TREX2"
}